{
  "term_id": "UNKNOWN:0001",
  "gene_symbol": "UMOD",
  "gene_name": "Uromodulin",
  "gene": "UniProtKB:P07911",
  "term_label": "Unknown molecular function"
}